phytochelatin biosynthetic process [GO:0046938] (BP) Definition: The chemical reactions and pathways resulting in the formation of phytochelatins, any of a group of peptides that bind metals (Cd, Zn, Cu, Pb, Hg) in thiolate coordination complexes. The structure is of the type (gamma-glutamyl-cysteinyl)n-glycine, where n is 2 to 11. Relationships: is a type of GO:0043604; is a type of GO:0046937 Also known as: phytochelatin anabolism, phytochelatin biosynthesis, phytochelatin formation, phytochelatin synthesis, cadystin biosynthetic process Sources: ISBN:0198506732